{
  "gene": "UniProtKB:P51911",
  "term_label": "actin filament organization",
  "gene_symbol": "CNN1",
  "gene_name": "Calponin-1",
  "term_id": "GO:0007015"
}